RNA polymerase II CTD heptapeptide repeat T4 phosphatase activity [GO:0180005] (molecular function) Definition: Catalysis of the reaction: RNA polymerase II large subunit CTD heptapeptide repeat--phospho-L-threonine (consensus YSPTSPS)(position 4) + H2O = RNA polymerase II large subunit + phosphate. References: PMID:22622228 Also known as: RNA polymerase II C-terminal domain T4 phosphatase activity Relationships: is a type of RNA polymerase II CTD heptapeptide repeat phosphatase activity [GO:0008420]